{
  "gene": "UniProtKB:P07437",
  "gene_symbol": "TUBB",
  "gene_name": "Tubulin beta chain",
  "term_id": "GO:0005200",
  "term_label": "structural constituent of cytoskeleton"
}